{
  "gene_symbol": "ANKMY2",
  "term_label": "Unknown cellular component",
  "term_id": "UNKNOWN:0003",
  "gene": "UniProtKB:Q8IV38",
  "gene_name": "Ankyrin repeat and MYND domain-containing protein 2"
}